{
  "gene": "UniProtKB:P01824",
  "gene_symbol": "IGHV4-39",
  "term_label": "antigen binding",
  "term_id": "GO:0003823",
  "gene_name": "Immunoglobulin heavy variable 4-39"
}